{
  "term_id": "GO:0000045",
  "gene_symbol": "RAB1B",
  "term_label": "autophagosome assembly",
  "gene_name": "Ras-related protein Rab-1B",
  "gene": "UniProtKB:Q9H0U4"
}